{
  "term_label": "Unknown biological process",
  "gene": "UniProtKB:Q9NQE9",
  "term_id": "UNKNOWN:0002",
  "gene_name": "Adenosine 5'-monophosphoramidase HINT3",
  "gene_symbol": "HINT3"
}